{
  "term_id": "GO:0015937",
  "gene_name": "Dephospho-CoA kinase domain-containing protein",
  "gene_symbol": "DCAKD",
  "gene": "UniProtKB:Q8WVC6",
  "term_label": "coenzyme A biosynthetic process"
}